{
  "gene_name": "Junctional adhesion molecule A",
  "term_id": "GO:0090559",
  "gene": "UniProtKB:Q9Y624",
  "term_label": "regulation of membrane permeability",
  "gene_symbol": "F11R"
}